macropinosome lysis involved in viral entry into host cell [GO:0075511] (biological process) Sources: GOC:bf, GOC:jl Relationships: is a type of lysis of host organelle involved in viral entry into host cell [GO:0039664] Definition: Viral-induced lysis of the macropinosome involved in the uptake of a virus into a host cell. Occurs after internalization of the virus in a macropinosome, and results in the release of viral contents from the macropinosome into the host cell cytoplasm.